cellular response to acidic pH [GO:0071468] (BP) Sources: GOC:go_curators, GOC:mah, Wikipedia:PH Also known as: cellular response to acidity Note: This term should be used to annotate instances where a cell is responding to a chemical that is playing the role of an acid (e.g. proton donor) and therefore lowering the pH. If instead you wish to describe a response to a specific acid as a chemical, such as the anion portion of glutamate, please annotate to the appropriate child of GO:0071229 'cellular response to acid chemical'. Relationships: is a type of response to acidic pH [GO:0010447]; is a type of cellular response to pH [GO:0071467] Definition: Any process that results in a change in state or activity of a cell (in terms of movement, secretion, enzyme production, gene expression, etc.) as a result of a pH stimulus with pH < 7. pH is a measure of the acidity or basicity of an aqueous solution. Subtypes: GO:1990451